{
  "term_label": "negative regulation of T cell receptor signaling pathway",
  "term_id": "GO:0050860",
  "gene_name": "Ubiquitin-associated and SH3 domain-containing protein A",
  "gene_symbol": "UBASH3A",
  "gene": "UniProtKB:P57075"
}